molybdate ion export from vacuole [GO:0090414] (biological process) Relationships: is a type of GO:0015689; is a type of vacuolar transmembrane transport [GO:0034486] Sources: GOC:tb Definition: The directed movement of molybdate ions out of the vacuole.